{
  "gene_name": "Protein phosphatase 1 regulatory inhibitor subunit 16B",
  "gene": "UniProtKB:Q96T49",
  "term_id": "GO:1903670",
  "gene_symbol": "PPP1R16B",
  "term_label": "regulation of sprouting angiogenesis"
}